{
  "gene_name": "Transcription regulator protein BACH2",
  "term_label": "regulation of transcription by RNA polymerase II",
  "term_id": "GO:0006357",
  "gene_symbol": "BACH2",
  "gene": "UniProtKB:Q9BYV9"
}